{
  "term_label": "cytoplasm",
  "gene_symbol": "HENMT1",
  "gene_name": "Small RNA 2'-O-methyltransferase",
  "term_id": "GO:0005737",
  "gene": "UniProtKB:Q5T8I9"
}